{
  "gene_name": "FOXL2 neighbor protein",
  "term_id": "UNKNOWN:0001",
  "gene_symbol": "FOXL2NB",
  "term_label": "Unknown molecular function",
  "gene": "UniProtKB:Q6ZUU3"
}